{
  "gene_name": "Lathosterol oxidase",
  "term_id": "GO:0000248",
  "gene": "UniProtKB:O75845",
  "term_label": "C-5 sterol desaturase activity",
  "gene_symbol": "SC5D"
}